{
  "gene_name": "Small ubiquitin-related modifier 4",
  "gene": "UniProtKB:Q6EEV6",
  "gene_symbol": "SUMO4",
  "term_label": "nucleus",
  "term_id": "GO:0005634"
}